trabecula formation [GO:0060343] (biological process) Subtypes: liver trabecula formation [GO:0060344], GO:0060345, bone trabecula formation [GO:0060346], heart trabecula formation [GO:0060347] Definition: The process of creating a trabecula in an organ. A trabecula is a small, often microscopic, tissue element in the form of a small beam, strut or rod, which generally has a mechanical function. Trabecula are usually but not necessarily, composed of dense collagenous tissue. Sources: GOC:dph Also known as: trabeculation, trabecula biogenesis Relationships: is_a anatomical structure formation involved in morphogenesis [GO:0048646]; is part of animal organ morphogenesis [GO:0009887]; BFO_0000050 trabecula morphogenesis [GO:0061383]